{
  "gene_name": "WASH complex subunit 2C",
  "term_id": "GO:0036010",
  "gene": "UniProtKB:Q9Y4E1",
  "gene_symbol": "WASHC2C",
  "term_label": "protein localization to endosome"
}